{
  "term_id": "UNKNOWN:0003",
  "gene_symbol": "TMPO",
  "gene_name": "Lamina-associated polypeptide 2, isoform alpha",
  "gene": "UniProtKB:P42166",
  "term_label": "Unknown cellular component"
}